{
  "term_label": "DNA-binding transcription repressor activity, RNA polymerase II-specific",
  "gene": "UniProtKB:Q9Y2W7",
  "gene_symbol": "KCNIP3",
  "term_id": "GO:0001227",
  "gene_name": "Calsenilin"
}